{
  "term_id": "GO:0005856",
  "gene_name": "Keratin, type I cytoskeletal 13",
  "gene_symbol": "KRT13",
  "gene": "UniProtKB:P13646",
  "term_label": "cytoskeleton"
}